{
  "gene_name": "Ras GTPase-activating protein 3",
  "gene": "UniProtKB:Q14644",
  "term_id": "GO:1902531",
  "term_label": "regulation of intracellular signal transduction",
  "gene_symbol": "RASA3"
}